cerebral cortex radially oriented cell migration [GO:0021799] (biological process) Definition: The migration of cells in the developing cerebral cortex in which cells move from the ventricular and/or subventricular zone toward the surface of the brain. Subtypes: cerebral cortex radial glia-guided migration [GO:0021801], somal translocation [GO:0021802] References: PMID:12626695 Sources: GOC:cls, GOC:dgh, GOC:dph, GOC:jid, GO_REF:0000021 Relationships: is a type of cerebral cortex cell migration [GO:0021795]